{
  "term_id": "GO:0005634",
  "term_label": "nucleus",
  "gene": "UniProtKB:Q99741",
  "gene_name": "Cell division control protein 6 homolog",
  "gene_symbol": "CDC6"
}